metal ion sensor activity [GO:0140784] (molecular function) Sources: GOC:pg Relationships: is a type of molecular sensor activity [GO:0140299] Definition: Binding to and responding, e.g. by conformational change, to changes in the cellular level of a metal ion. Subtypes: calcium ion sensor activity [GO:0061891], cadmium ion sensor activity [GO:0097063], copper ion sensor activity [GO:0097077], zinc ion sensor activity [GO:0106219], iron sensor activity [GO:0140482]